{
  "gene": "UniProtKB:Q9Y3T9",
  "term_label": "histone binding",
  "term_id": "GO:0042393",
  "gene_name": "Nucleolar complex protein 2 homolog",
  "gene_symbol": "NOC2L"
}